{
  "term_label": "cytokine activity",
  "term_id": "GO:0005125",
  "gene": "UniProtKB:Q7Z5Y6",
  "gene_symbol": "BMP8A",
  "gene_name": "Bone morphogenetic protein 8A"
}